{
  "gene_symbol": "DNAH9",
  "gene": "UniProtKB:Q9NYC9",
  "term_label": "9+2 motile cilium",
  "gene_name": "Dynein axonemal heavy chain 9",
  "term_id": "GO:0097729"
}